{
  "term_label": "immunoglobulin complex",
  "gene_symbol": "IGKV2-28",
  "term_id": "GO:0019814",
  "gene": "UniProtKB:A0A075B6P5",
  "gene_name": "Immunoglobulin kappa variable 2-28"
}